{
  "gene": "UniProtKB:Q5JUW0",
  "term_id": "GO:0000122",
  "gene_name": "KRAB domain-containing protein 4",
  "gene_symbol": "KRBOX4",
  "term_label": "negative regulation of transcription by RNA polymerase II"
}